beta-elemene synthase activity [GO:0102889] (molecular function) Definition: Catalysis of the reaction: 2-trans,6-trans-farnesyl diphosphate = beta-elemene + diphosphoric acid. Relationships: is a type of carbon-oxygen lyase activity, acting on phosphates [GO:0016838] Sources: MetaCyc:RXN-8432